{
  "term_label": "signaling receptor activity",
  "gene_name": "TLR4 interactor with leucine rich repeats",
  "term_id": "GO:0038023",
  "gene": "UniProtKB:Q7L0X0",
  "gene_symbol": "TRIL"
}